prostaglandin transport [GO:0015732] (biological process) Definition: The directed movement of prostaglandins into, out of or within a cell, or between cells, by means of some agent such as a transporter or pore. Sources: GOC:krc Relationships: is a type of fatty acid transport [GO:0015908]; is a type of GO:0071715 Subtypes: prostaglandin secretion [GO:0032310], sodium-independent prostaglandin transport [GO:0071720]